{
  "term_label": "Unknown cellular component",
  "term_id": "UNKNOWN:0003",
  "gene_symbol": "ABHD16A",
  "gene_name": "Phosphatidylserine lipase ABHD16A",
  "gene": "UniProtKB:O95870"
}